{
  "gene_symbol": "NCF1",
  "gene_name": "Neutrophil cytosol factor 1",
  "term_id": "GO:0005737",
  "gene": "UniProtKB:P14598",
  "term_label": "cytoplasm"
}